{
  "term_id": "GO:0004984",
  "term_label": "olfactory receptor activity",
  "gene_name": "Olfactory receptor 5H15",
  "gene": "UniProtKB:A6NDH6",
  "gene_symbol": "OR5H15"
}